{
  "term_id": "GO:0099502",
  "gene": "UniProtKB:Q14184",
  "gene_name": "Double C2-like domain-containing protein beta",
  "gene_symbol": "DOC2B",
  "term_label": "calcium-dependent activation of synaptic vesicle fusion"
}